{
  "gene": "UniProtKB:P59534",
  "gene_symbol": "TAS2R39",
  "term_id": "GO:0001580",
  "gene_name": "Taste receptor type 2 member 39",
  "term_label": "detection of chemical stimulus involved in sensory perception of bitter taste"
}